cellular response to lipid hydroperoxide [GO:0071449] (biological process) Relationships: is a type of response to lipid hydroperoxide [GO:0006982]; is a type of GO:0071396; is a type of cellular response to hydroperoxide [GO:0071447] Definition: Any process that results in a change in state or activity of a cell (in terms of movement, secretion, enzyme production, gene expression, etc.) as a result of a lipid hydroperoxide stimulus. Lipid hydroperoxide is the highly reactive primary oxygenated products of polyunsaturated fatty acids. Also known as: cellular response to LHPO Sources: GOC:mah